{
  "gene_symbol": "KMT2D",
  "term_id": "GO:0045944",
  "gene": "UniProtKB:O14686",
  "gene_name": "Histone-lysine N-methyltransferase 2D",
  "term_label": "positive regulation of transcription by RNA polymerase II"
}